{
  "gene_name": "Cilia- and flagella-associated protein 144",
  "gene_symbol": "CFAP144",
  "term_id": "GO:0097546",
  "term_label": "ciliary base",
  "gene": "UniProtKB:A6NL82"
}